{
  "term_label": "adherens junction",
  "term_id": "GO:0005912",
  "gene": "UniProtKB:P55289",
  "gene_symbol": "CDH12",
  "gene_name": "Cadherin-12"
}